mitotic spindle pole body localization [GO:1990608] (biological process) Subtypes: mitotic spindle pole body insertion into the nuclear envelope [GO:0140480] Relationships: is a type of spindle pole body localization [GO:0070631]; is a type of mitotic cell cycle process [GO:1903047] Also known as: establishment and maintenance of spindle pole body localization, establishment of spindle pole body localisation, establishment of spindle pole body localization, mitotic spindle pole body localization to nuclear envelope, spindle pole body docking, spindle pole body localisation in nuclear envelope, spindle pole body localization in nuclear envelope, spindle pole body localization to nuclear envelope, spindle pole body positioning Definition: A process in which a mitotic spindle pole body is transported to, or maintained in, a specific cellular location. References: PMID:24963130